{
  "term_id": "GO:0006357",
  "term_label": "regulation of transcription by RNA polymerase II",
  "gene_name": "Cyclic AMP-dependent transcription factor ATF-6 beta",
  "gene_symbol": "ATF6B",
  "gene": "UniProtKB:Q99941"
}